lung secretory cell differentiation [GO:0061140] (biological process) Definition: The process in which a relatively unspecialized cell acquires specialized features of a lung secretory cell. A lung secretory cell is a specialized epithelial cell of the lung that contains large secretory granules in its apical part. Sources: GOC:dph Subtypes: GO:0060480, type II pneumocyte differentiation [GO:0060510], lung neuroendocrine cell differentiation [GO:0061100] Relationships: is a type of lung epithelial cell differentiation [GO:0060487]